{
  "gene": "UniProtKB:Q7Z4L0",
  "term_id": "UNKNOWN:0001",
  "gene_symbol": "COX8C",
  "gene_name": "Cytochrome c oxidase subunit 8C, mitochondrial",
  "term_label": "Unknown molecular function"
}